regulation of cell proliferation involved in heart morphogenesis [GO:2000136] (biological process) Definition: Any process that modulates the frequency, rate or extent of cell proliferation involved in heart morphogenesis. Relationships: is a type of regulation of cell population proliferation [GO:0042127]; regulates cell proliferation involved in heart morphogenesis [GO:0061323] Subtypes: GO:0003250, GO:0003264, regulation of cell proliferation involved in outflow tract morphogenesis [GO:1901963], negative regulation of cell proliferation involved in heart morphogenesis [GO:2000137], positive regulation of cell proliferation involved in heart morphogenesis [GO:2000138] Sources: GOC:dph